{
  "term_label": "channel activity",
  "gene_symbol": "BCL2",
  "gene_name": "Apoptosis regulator Bcl-2",
  "gene": "UniProtKB:P10415",
  "term_id": "GO:0015267"
}